positive regulation of nuclear-transcribed mRNA poly(A) tail shortening [GO:0060213] (biological process) Also known as: positive regulation of 3' to 5' mRNA deadenylation, positive regulation of mRNA deadenylation, positive regulation of nuclear mRNA poly(A) tail shortening Definition: Any process that increases the frequency, rate or extent of poly(A) tail shortening of a nuclear-transcribed mRNA. Poly(A) tail shortening is the decrease in length of the poly(A) tail of an mRNA from full length to an oligo(A) length. Relationships: is a type of regulation of nuclear-transcribed mRNA poly(A) tail shortening [GO:0060211]; is a type of GO:0061014; positively regulates nuclear-transcribed mRNA poly(A) tail shortening [GO:0000289] Sources: GOC:dph, GOC:tb